response to high fluence blue light stimulus by blue high-fluence system [GO:0055121] (biological process) Sources: GOC:mtg_far_red Also known as: response to high fluence blue light, response to high fluence blue light by bhf system Relationships: is a type of GO:0009637; is_a response to high light intensity [GO:0009644] Definition: Any process that results in a change in state or activity of a cell or an organism (in terms of movement, secretion, enzyme production, gene expression, etc.) as a result of the detection of a high fluence blue light stimulus by the blue high-fluence system. Blue light is electromagnetic radiation with a wavelength of between 440 and 500nm. The blue high-fluence system responds to blue light at levels between 100 and 1000 micromols/m2.